{
  "term_id": "GO:0007167",
  "gene": "UniProtKB:Q8WWN9",
  "gene_symbol": "IPCEF1",
  "term_label": "enzyme-linked receptor protein signaling pathway",
  "gene_name": "Interactor protein for cytohesin exchange factors 1"
}